{
  "gene_name": "Olfactory receptor 11L1",
  "term_label": "odorant binding",
  "term_id": "GO:0005549",
  "gene": "UniProtKB:Q8NGX0",
  "gene_symbol": "OR11L1"
}